{
  "gene": "UniProtKB:Q53GG5",
  "term_id": "GO:0003779",
  "gene_name": "PDZ and LIM domain protein 3",
  "term_label": "actin binding",
  "gene_symbol": "PDLIM3"
}